{
  "gene": "UniProtKB:Q96FE7",
  "term_id": "GO:0005615",
  "term_label": "extracellular space",
  "gene_symbol": "PIK3IP1",
  "gene_name": "Phosphoinositide-3-kinase-interacting protein 1"
}